{
  "term_id": "UNKNOWN:0003",
  "gene_symbol": "LOC122455340",
  "term_label": "Unknown cellular component",
  "gene": "UniProtKB:A0A1B0GVY2",
  "gene_name": "Uncharacterized protein"
}